regulation of protein catabolic process at postsynapse, modulating synaptic transmission [GO:0099576] (biological process) Note: Note that this term was created for the SynGO project, and will be obsoleted when the SynGO annotations are made in Noctua. Relationships: is a type of regulation of protein catabolic process [GO:0042176]; is a type of GO:0099170 Sources: GOC:dos Definition: Any process that modulates synaptic transmission by regulating a catabolic process occurring at a postsynapse.